regulation of interleukin-27-mediated signaling pathway [GO:0070107] (biological process) Definition: Any process that modulates the rate, frequency or extent of an interleukin-27-mediated signaling pathway. Relationships: is a type of regulation of cytokine-mediated signaling pathway [GO:0001959]; regulates GO:0070106 Subtypes: negative regulation of interleukin-27-mediated signaling pathway [GO:0070108], positive regulation of interleukin-27-mediated signaling pathway [GO:0070109] Also known as: regulation of IL-27-mediated signaling pathway, regulation of IL27RA/IL6ST signaling pathway, regulation of interleukin-27-mediated signalling pathway Sources: GOC:BHF, GOC:mah